{
  "gene": "UniProtKB:Q7Z4V5",
  "term_id": "GO:0062072",
  "gene_name": "Hepatoma-derived growth factor-related protein 2",
  "gene_symbol": "HDGFL2",
  "term_label": "histone H3K9me2/3 reader activity"
}